{
  "gene": "UniProtKB:A8MVW5",
  "gene_name": "HEPACAM family member 2",
  "term_id": "GO:0030496",
  "term_label": "midbody",
  "gene_symbol": "HEPACAM2"
}